centrosome localization [GO:0051642] (biological process) Relationships: is a type of GO:0061842 Sources: GOC:ai Subtypes: establishment of centrosome localization [GO:0051660], maintenance of centrosome location [GO:0051661] Also known as: centrosome localisation, establishment and maintenance of centrosome localization Definition: Any process in which a centrosome is transported to, and/or maintained in, a specific location within the cell.